{
  "term_label": "nucleus",
  "term_id": "GO:0005634",
  "gene_symbol": "KPNA3",
  "gene": "UniProtKB:O00505",
  "gene_name": "Importin subunit alpha-4"
}